{
  "term_label": "signal transduction",
  "gene_symbol": "CNTNAP3B",
  "term_id": "GO:0007165",
  "gene_name": "Contactin-associated protein-like 3B",
  "gene": "UniProtKB:Q96NU0"
}